{
  "gene_name": "Granzyme K",
  "term_label": "granzyme-mediated programmed cell death signaling pathway",
  "term_id": "GO:0140507",
  "gene_symbol": "GZMK",
  "gene": "UniProtKB:P49863"
}